{
  "term_label": "ubiquinone biosynthetic process",
  "term_id": "GO:0006744",
  "gene_name": "NADH dehydrogenase [ubiquinone] 1 alpha subcomplex subunit 9, mitochondrial",
  "gene": "UniProtKB:Q16795",
  "gene_symbol": "NDUFA9"
}